{
  "gene_symbol": "SPACA6",
  "term_label": "Unknown cellular component",
  "gene_name": "Sperm acrosome membrane-associated protein 6",
  "term_id": "UNKNOWN:0003",
  "gene": "UniProtKB:W5XKT8"
}